{
  "gene": "UniProtKB:Q13442",
  "term_label": "Unknown molecular function",
  "gene_name": "28 kDa heat- and acid-stable phosphoprotein",
  "gene_symbol": "PDAP1",
  "term_id": "UNKNOWN:0001"
}